{
  "gene_symbol": "MIEN1",
  "term_label": "cytosol",
  "gene_name": "Migration and invasion enhancer 1",
  "term_id": "GO:0005829",
  "gene": "UniProtKB:Q9BRT3"
}